citramalate lyase activity [GO:0047776] (molecular function) Relationships: is a type of oxo-acid-lyase activity [GO:0016833] Definition: Catalysis of the reaction: S-citramalate = acetate + pyruvate. Sources: EC:4.1.3.22, RHEA:15545 Also known as: (+)-citramalate pyruvate-lyase activity, (3S)-citramalate pyruvate-lyase (acetate-forming), (3S)-citramalate pyruvate-lyase activity, (S)-citramalate lyase activity, citramalate pyruvate lyase activity, citramalate pyruvate-lyase activity, citramalate synthetase activity, citramalic synthase activity, citramalic-condensing enzyme